{
  "gene_name": "Protein ZGRF1",
  "term_label": "site of double-strand break",
  "gene_symbol": "ZGRF1",
  "term_id": "GO:0035861",
  "gene": "UniProtKB:Q86YA3"
}